{
  "term_id": "GO:0005085",
  "gene": "UniProtKB:O95267",
  "gene_name": "RAS guanyl-releasing protein 1",
  "term_label": "guanyl-nucleotide exchange factor activity",
  "gene_symbol": "RASGRP1"
}